{
  "gene": "UniProtKB:Q969V1",
  "term_id": "GO:0004966",
  "gene_name": "Melanin-concentrating hormone receptor 2",
  "term_label": "galanin receptor activity",
  "gene_symbol": "MCHR2"
}